{
  "term_id": "GO:0032051",
  "gene_symbol": "HIP1",
  "gene": "UniProtKB:O00291",
  "gene_name": "Huntingtin-interacting protein 1",
  "term_label": "clathrin light chain binding"
}